{
  "gene": "UniProtKB:Q6P589",
  "gene_name": "Tumor necrosis factor alpha-induced protein 8-like protein 2",
  "term_id": "UNKNOWN:0001",
  "term_label": "Unknown molecular function",
  "gene_symbol": "TNFAIP8L2"
}